{
  "gene": "UniProtKB:O60397",
  "term_id": "GO:0006119",
  "gene_name": "Putative cytochrome c oxidase subunit 7A3, mitochondrial",
  "gene_symbol": "COX7A2P2",
  "term_label": "oxidative phosphorylation"
}